{
  "term_id": "GO:0019955",
  "gene": "UniProtKB:P78552",
  "gene_symbol": "IL13RA1",
  "gene_name": "Interleukin-13 receptor subunit alpha-1",
  "term_label": "cytokine binding"
}